{
  "gene_symbol": "A0A8I5KYS1",
  "term_id": "UNKNOWN:0002",
  "term_label": "Unknown biological process",
  "gene_name": "Vegetative cell wall protein gp1-like",
  "gene": "UniProtKB:A0A8I5KYS1"
}